high-density lipoprotein particle remodeling [GO:0034375] (biological process) Definition: The acquisition, loss or modification of a protein or lipid within a high-density lipoprotein particle, including the hydrolysis of triglyceride by hepatic lipase, with the subsequent loss of free fatty acid, and the transfer of cholesterol esters from LDL to a triglyceride-rich lipoprotein particle by cholesteryl ester transfer protein (CETP), with the simultaneous transfer of triglyceride to LDL. Sources: GOC:BHF, GOC:expert_pt, GOC:mah, GOC:rl Also known as: HDL remodeling, HDL remodelling, high-density lipoprotein particle remodelling Relationships: is a type of plasma lipoprotein particle remodeling [GO:0034369] Subtypes: conversion of discoidal high-density lipoprotein particle to spherical high-density lipoprotein particle [GO:0034376]